{
  "term_id": "GO:0005886",
  "gene": "UniProtKB:Q96QD8",
  "term_label": "plasma membrane",
  "gene_name": "Sodium-coupled neutral amino acid symporter 2",
  "gene_symbol": "SLC38A2"
}